{
  "term_id": "GO:0001676",
  "gene": "UniProtKB:O14975",
  "gene_name": "Long-chain fatty acid transport protein 2",
  "gene_symbol": "SLC27A2",
  "term_label": "long-chain fatty acid metabolic process"
}